{
  "gene_symbol": "GCC2",
  "gene_name": "GRIP and coiled-coil domain-containing protein 2",
  "gene": "UniProtKB:Q8IWJ2",
  "term_label": "trans-Golgi network",
  "term_id": "GO:0005802"
}